2-deoxystreptamine glucosyltransferase activity [GO:0102318] (MF) Definition: Catalysis of the reaction: 2-deoxystreptamine + UDP-alpha-D-glucose = 2'-deamino-2'-hydroxyparomamine + UDP(3-) + H+. Sources: EC:2.4.1.284, GOC:pz Relationships: is a type of hexosyltransferase activity [GO:0016758]